{
  "term_id": "GO:0022625",
  "gene_symbol": "RPL27A",
  "gene_name": "Large ribosomal subunit protein uL15",
  "term_label": "cytosolic large ribosomal subunit",
  "gene": "UniProtKB:P46776"
}